{
  "gene_symbol": "MYL7",
  "term_label": "calcium ion binding",
  "term_id": "GO:0005509",
  "gene_name": "Myosin regulatory light chain 2, atrial isoform",
  "gene": "UniProtKB:Q01449"
}